{
  "term_label": "RNA binding",
  "gene": "UniProtKB:Q7L8L6",
  "gene_symbol": "FASTKD5",
  "gene_name": "FAST kinase domain-containing protein 5, mitochondrial",
  "term_id": "GO:0003723"
}